austinol biosynthetic process [GO:1900560] (biological process) Definition: The chemical reactions and pathways resulting in the formation of austinol. Sources: GOC:TermGenie, GOC:di Regulation: regulated by regulation of austinol biosynthetic process [GO:1900640]; negatively regulated by GO:1900641; positively regulated by GO:1900642 Relationships: is_a GO:0009058 Also known as: austinol anabolism, austinol biosynthesis, austinol formation, austinol synthesis